{
  "gene_name": "Barrier-to-autointegration factor",
  "gene_symbol": "BANF1",
  "term_label": "nucleus",
  "gene": "UniProtKB:O75531",
  "term_id": "GO:0005634"
}